{
  "gene_symbol": "PDZD7",
  "term_label": "sensory perception of sound",
  "gene": "UniProtKB:Q9H5P4",
  "term_id": "GO:0007605",
  "gene_name": "PDZ domain-containing protein 7"
}